{
  "term_id": "UNKNOWN:0001",
  "term_label": "Unknown molecular function",
  "gene": "UniProtKB:Q96AA8",
  "gene_name": "Janus kinase and microtubule-interacting protein 2",
  "gene_symbol": "JAKMIP2"
}